{
  "gene": "UniProtKB:Q96KW2",
  "gene_symbol": "POM121L2",
  "term_id": "GO:0006405",
  "gene_name": "POM121-like protein 2",
  "term_label": "RNA export from nucleus"
}